{
  "gene_symbol": "ALPK1",
  "term_id": "GO:0048029",
  "term_label": "monosaccharide binding",
  "gene_name": "Alpha-protein kinase 1",
  "gene": "UniProtKB:Q96QP1"
}